uterine smooth muscle relaxation [GO:0044558] (biological process) Regulation: regulated by regulation of uterine smooth muscle relaxation [GO:1900719]; negatively regulated by negative regulation of uterine smooth muscle relaxation [GO:1900720]; positively regulated by positive regulation of uterine smooth muscle relaxation [GO:1900721] Also known as: smooth muscle relaxation of the uterus Sources: GOC:jl Relationships: is_a relaxation of smooth muscle [GO:0044557] Definition: A process in which the extent of smooth muscle contraction is reduced in the uterus.